{
  "gene_name": "Endothelial PAS domain-containing protein 1",
  "term_label": "lung development",
  "gene": "UniProtKB:Q99814",
  "term_id": "GO:0030324",
  "gene_symbol": "EPAS1"
}